positive regulation of adenosine transport [GO:0032251] (biological process) Definition: Any process that activates or increases the frequency, rate or extent of the directed movement of adenosine into, out of or within a cell, or between cells, by means of some agent such as a transporter or pore. Relationships: is_a GO:0032248; is a type of regulation of adenosine transport [GO:0032249]; positively regulates adenosine transport [GO:0032238] Sources: GOC:mah Also known as: up regulation of adenosine transport, up-regulation of adenosine transport, upregulation of adenosine transport, activation of adenosine transport, stimulation of adenosine transport